{
  "gene_name": "Taste receptor type 2 member 43",
  "gene": "UniProtKB:P59537",
  "term_id": "GO:0033038",
  "gene_symbol": "TAS2R43",
  "term_label": "bitter taste receptor activity"
}